{
  "gene_symbol": "VDAC2",
  "gene_name": "Voltage-dependent anion-selective channel protein 2",
  "gene": "UniProtKB:P45880",
  "term_id": "GO:0008308",
  "term_label": "voltage-gated monoatomic anion channel activity"
}